{
  "gene": "UniProtKB:P54852",
  "term_id": "GO:0005886",
  "gene_symbol": "EMP3",
  "gene_name": "Epithelial membrane protein 3",
  "term_label": "plasma membrane"
}